compound eye photoreceptor fate commitment [GO:0001752] (biological process) Definition: The process in which the developmental fate of a cell becomes restricted such that it will develop into a compound eye photoreceptor cell. A photoreceptor cell is a cell that responds to incident electromagnetic radiation. Different classes of photoreceptor have different spectral sensitivities and express different photosensitive pigments. Sources: GOC:mtg_sensu Relationships: is a type of eye photoreceptor cell fate commitment [GO:0042706]; is part of compound eye photoreceptor cell differentiation [GO:0001751] Subtypes: R8 cell fate commitment [GO:0007460], R1/R6 cell fate commitment [GO:0007462], R2/R5 cell fate commitment [GO:0007463], R3/R4 cell fate commitment [GO:0007464], R7 cell fate commitment [GO:0007465]